{
  "term_label": "cristae formation",
  "gene_symbol": "DNAJC11",
  "term_id": "GO:0042407",
  "gene_name": "DnaJ homolog subfamily C member 11",
  "gene": "UniProtKB:Q9NVH1"
}